integrin alphaX-beta2 complex [GO:0034689] (CC) Also known as: alphaX-beta2 integrin complex, Itgax-Itgb2 complex Definition: An integrin complex that comprises one alphaX subunit and one beta2 subunit. Relationships: is a type of GO:0008305 References: PMID:12297042